{
  "gene": "UniProtKB:A6NNM8",
  "term_id": "GO:0015631",
  "gene_name": "Tubulin polyglutamylase TTLL13",
  "term_label": "tubulin binding",
  "gene_symbol": "TTLL13"
}